{
  "gene": "UniProtKB:O76015",
  "term_label": "intermediate filament organization",
  "gene_name": "Keratin, type I cuticular Ha8",
  "gene_symbol": "KRT38",
  "term_id": "GO:0045109"
}